keto-D-gluconate catabolic process [GO:0019524] (biological process) Also known as: keto-D-gluconate breakdown, keto-D-gluconate catabolism, keto-D-gluconate degradation Sources: ISBN:0198506732 Definition: The chemical reactions and pathways resulting in the breakdown of keto-D-gluconate, the anion of keto-D-gluconic acid, an aldonic acid derived from glucose. Relationships: is a type of ketogluconate catabolic process [GO:0046181]